{
  "gene_symbol": "OR52B6",
  "term_id": "UNKNOWN:0002",
  "term_label": "Unknown biological process",
  "gene": "UniProtKB:Q8NGF0",
  "gene_name": "Olfactory receptor 52B6"
}